{
  "gene": "UniProtKB:Q9H1E1",
  "term_label": "defense response to fungus",
  "gene_symbol": "RNASE7",
  "term_id": "GO:0050832",
  "gene_name": "Ribonuclease 7"
}